{
  "gene_symbol": "KIF3B",
  "gene": "UniProtKB:O15066",
  "term_label": "kinesin complex",
  "gene_name": "Kinesin-like protein KIF3B",
  "term_id": "GO:0005871"
}